{
  "gene": "UniProtKB:Q96P65",
  "term_id": "GO:0007186",
  "gene_name": "Pyroglutamylated RF-amide peptide receptor",
  "gene_symbol": "QRFPR",
  "term_label": "G protein-coupled receptor signaling pathway"
}